{
  "term_label": "anterograde dendritic transport of neurotransmitter receptor complex",
  "gene_name": "Kinesin heavy chain isoform 5C",
  "gene": "UniProtKB:O60282",
  "gene_symbol": "KIF5C",
  "term_id": "GO:0098971"
}